3-cyano-L-alanine biosynthetic process [GO:1903560] (biological process) Definition: The chemical reactions and pathways resulting in the formation of 3-cyano-L-alanine. Also known as: 3-cyano-L-alanine anabolism, 3-cyano-L-alanine biosynthesis, 3-cyano-L-alanine formation, 3-cyano-L-alanine synthesis Relationships: is a type of nitrile biosynthetic process [GO:0080028]; is a type of L-amino acid biosynthetic process [GO:0170034]; is a type of non-proteinogenic amino acid biosynthetic process [GO:0170043] References: PMID:24100226, PMID:24843024 Sources: GOC:TermGenie, GOC:kmv, GO_REF:0000068